{
  "gene_symbol": "KCNA3",
  "term_label": "potassium ion transmembrane transport",
  "gene_name": "Potassium voltage-gated channel subfamily A member 3",
  "term_id": "GO:0071805",
  "gene": "UniProtKB:P22001"
}